{
  "gene_symbol": "SPP1",
  "gene_name": "Osteopontin",
  "gene": "UniProtKB:P10451",
  "term_id": "GO:0045780",
  "term_label": "positive regulation of bone resorption"
}